negative regulation of T cell tolerance induction [GO:0002665] (biological process) Also known as: down regulation of T cell tolerance induction, down-regulation of T cell tolerance induction, downregulation of T cell tolerance induction, negative regulation of T lymphocyte tolerance induction, negative regulation of T-cell tolerance induction, negative regulation of T-lymphocyte tolerance induction, inhibition of T cell tolerance induction Subtypes: negative regulation of T cell anergy [GO:0002668], negative regulation of peripheral T cell tolerance induction [GO:0002850] Sources: GOC:add Definition: Any process that stops, prevents, or reduces the frequency, rate, or extent of T cell tolerance induction. Relationships: is a type of GO:0002644; is a type of regulation of T cell tolerance induction [GO:0002664]; RO_0002212 T cell tolerance induction [GO:0002517]